{
  "term_label": "maintenance of gastrointestinal epithelium",
  "gene_symbol": "TFF1",
  "gene": "UniProtKB:P04155",
  "gene_name": "Trefoil factor 1",
  "term_id": "GO:0030277"
}